{
  "gene_symbol": "STARD3NL",
  "term_label": "cholesterol binding",
  "term_id": "GO:0015485",
  "gene": "UniProtKB:O95772",
  "gene_name": "STARD3 N-terminal-like protein"
}